{
  "term_label": "Unknown molecular function",
  "gene_symbol": "CSN2",
  "term_id": "UNKNOWN:0001",
  "gene": "UniProtKB:P05814",
  "gene_name": "Beta-casein"
}